{
  "term_id": "GO:1903078",
  "gene_name": "SH3 and cysteine-rich domain-containing protein 2",
  "gene_symbol": "STAC2",
  "term_label": "positive regulation of protein localization to plasma membrane",
  "gene": "UniProtKB:Q6ZMT1"
}